chondroitin 6-sulfotransferase activity [GO:0008459] (MF) Relationships: is a type of GO:0034481 Also known as: chondroitin 6-sulphotransferase activity, 3'-phosphoadenosine 5'-phosphosulfate (PAPS):chondroitin sulfate sulfotransferase activity, 3'-phosphoadenylyl-sulfate:chondroitin 6'-sulfotransferase activity, chondroitin 6-O-sulfotransferase activity, terminal 6-sulfotransferase activity Sources: EC:2.8.2.17 Definition: Catalysis of the reaction: 3'-phosphoadenosine 5'-phosphosulfate + chondroitin = adenosine 3',5'-bisphosphate + chondroitin 6'-sulfate.